ovarian fusome organization [GO:0030723] (biological process) Sources: GOC:dph, GOC:jl, GOC:mah, ISBN:0879694238 Definition: A process that is carried out at the cellular level which results in the assembly, arrangement of constituent parts, or disassembly of the fusome of ovarian cells, an organelle derived from the spectrosome. It anchors the mitotic spindle pole to provide orientation during cystoblast cell divisions. Also known as: ovarian fusome organisation, ovarian fusome organization and biogenesis Relationships: is a type of fusome organization [GO:0045478]; is part of germarium-derived egg chamber formation [GO:0007293]